{
  "gene": "UniProtKB:Q6AHZ1",
  "term_label": "regulation of transcription by RNA polymerase II",
  "gene_name": "Zinc finger protein 518A",
  "term_id": "GO:0006357",
  "gene_symbol": "ZNF518A"
}